S-methyl-5-thioadenosine phosphorylase activity [GO:0017061] (molecular function) Also known as: 5'-methylthioadenosine phosphorylase activity, 5'-deoxy-5'-methylthioadenosine phosphorylase activity, 5'-methylthioadenosine:phosphate methylthio-D-ribosyl-transferase activity, MTA phosphorylase activity, MTAPase activity, MeSAdo phosphorylase activity, MeSAdo/Ado phosphorylase activity, S-methyl-5-thioadenosine:phosphate S-methyl-5-thio-alpha-D-ribosyl-transferase activity, methylthioadenosine nucleoside phosphorylase activity, methylthioadenosine phosphorylase activity Relationships: is a type of purine-nucleoside phosphorylase activity [GO:0004731] Sources: EC:2.4.2.28 Definition: Catalysis of the reaction: 5'-methylthioadenosine + phosphate = adenine + 5-methylthio-D-ribose 1-phosphate.